cellular response to peptide hormone stimulus [GO:0071375] (biological process) Subtypes: GO:0032869, cellular response to cholecystokinin [GO:0061848], GO:0071373, cellular response to corticotropin-releasing hormone stimulus [GO:0071376], cellular response to glucagon stimulus [GO:0071377], cellular response to growth hormone stimulus [GO:0071378], cellular response to gonadotropin-releasing hormone [GO:0097211], GO:1904117, cellular response to angiotensin [GO:1904385], GO:1905229, cellular response to insulin-like growth factor stimulus [GO:1990314], cellular response to prolactin [GO:1990646], GO:1990859, cellular response to gastrin [GO:1990878] Sources: GOC:mah Definition: Any process that results in a change in state or activity of a cell (in terms of movement, secretion, enzyme production, gene expression, etc.) as a result of a peptide hormone stimulus. A peptide hormone is any of a class of peptides that are secreted into the blood stream and have endocrine functions in living animals. Also known as: cellular response to polypeptide hormone stimulus Relationships: is a type of GO:0032870; is a type of response to peptide hormone [GO:0043434]; is a type of cellular response to nitrogen compound [GO:1901699]; is a type of GO:1901701